regulation of interleukin-1 production [GO:0032652] (biological process) Subtypes: GO:0032650, regulation of interleukin-1 beta production [GO:0032651], negative regulation of interleukin-1 production [GO:0032692], positive regulation of interleukin-1 production [GO:0032732] Definition: Any process that modulates the frequency, rate, or extent of interleukin-1 production. Also known as: regulation of IL-1 production, regulation of interleukin-1 biosynthetic process, regulation of interleukin-1 secretion Relationships: is a type of regulation of cytokine production [GO:0001817]; regulates interleukin-1 production [GO:0032612] Sources: GOC:mah